{
  "term_id": "GO:0030041",
  "gene": "UniProtKB:O75128",
  "term_label": "actin filament polymerization",
  "gene_symbol": "COBL",
  "gene_name": "Protein cordon-bleu"
}